{
  "gene": "UniProtKB:Q14469",
  "term_id": "GO:0005634",
  "gene_symbol": "HES1",
  "gene_name": "Transcription factor HES-1",
  "term_label": "nucleus"
}